{
  "gene": "UniProtKB:P40933",
  "term_id": "GO:0001819",
  "gene_name": "Interleukin-15",
  "gene_symbol": "IL15",
  "term_label": "positive regulation of cytokine production"
}